{
  "gene": "UniProtKB:Q9H0N0",
  "gene_name": "Ras-related protein Rab-6C",
  "term_label": "GTPase activity",
  "gene_symbol": "RAB6C",
  "term_id": "GO:0003924"
}